toluene catabolic process [GO:0042203] (biological process) Definition: The chemical reactions and pathways resulting in the breakdown of toluene, a volatile monoaromatic hydrocarbon found in crude petroleum and petroleum products. Sources: UM-BBD_pathwayID:tol Also known as: toluene breakdown, toluene catabolism, toluene degradation Relationships: is_a toluene metabolic process [GO:0018970]; is a type of xenobiotic catabolic process [GO:0042178]; is a type of GO:0072491; is a type of GO:0120253 Subtypes: anaerobic toluene catabolic process [GO:0046254] Regulation: regulated by regulation of toluene catabolic process [GO:1901434]; negatively regulated by GO:1901435; positively regulated by positive regulation of toluene catabolic process [GO:1901436]